{
  "term_id": "GO:0047498",
  "gene_symbol": "PLA2G2E",
  "term_label": "calcium-dependent phospholipase A2 activity",
  "gene_name": "Group IIE secretory phospholipase A2",
  "gene": "UniProtKB:Q9NZK7"
}